{
  "term_label": "L-amino acid transmembrane transporter activity",
  "term_id": "GO:0015179",
  "gene": "UniProtKB:Q9UM01",
  "gene_symbol": "SLC7A7",
  "gene_name": "Y+L amino acid transporter 1"
}